{
  "gene_name": "SH2B adapter protein 1",
  "term_label": "transmembrane receptor protein tyrosine kinase adaptor activity",
  "gene_symbol": "SH2B1",
  "term_id": "GO:0005068",
  "gene": "UniProtKB:Q9NRF2"
}